{
  "term_id": "GO:0061630",
  "gene_symbol": "TRIM13",
  "term_label": "ubiquitin protein ligase activity",
  "gene_name": "E3 ubiquitin-protein ligase TRIM13",
  "gene": "UniProtKB:O60858"
}